{
  "gene_symbol": "SMURF2",
  "term_id": "GO:0046332",
  "gene_name": "E3 ubiquitin-protein ligase SMURF2",
  "term_label": "SMAD binding",
  "gene": "UniProtKB:Q9HAU4"
}